neurohypophysis morphogenesis [GO:0048848] (biological process) Relationships: is a type of gland morphogenesis [GO:0022612]; is part of GO:0021985; is part of hypophysis morphogenesis [GO:0048850] Sources: GOC:cls, GOC:dgh, GOC:dph, GOC:jid Also known as: neurophysis morphogenesis, posterior pituitary gland morphogenesis, posterior pituitary morphogenesis Definition: The process in which the anatomical structures of the neurohypophysis are generated and organized. The neurohypophysis is the part of the pituitary gland that secretes hormones involved in blood pressure regulation.